negative regulation of isotype switching [GO:0045829] (biological process) Subtypes: negative regulation of isotype switching to IgE isotypes [GO:0048294], negative regulation of isotype switching to IgA isotypes [GO:0048297], GO:0048300, GO:0048303 Relationships: is a type of GO:0002638; is a type of negative regulation of immunoglobulin mediated immune response [GO:0002890]; is a type of regulation of isotype switching [GO:0045191]; is a type of GO:0045910; is a type of negative regulation of B cell activation [GO:0050869]; is a type of GO:0051093; negatively regulates isotype switching [GO:0045190] Sources: GOC:go_curators Definition: Any process that stops, prevents, or reduces the frequency, rate or extent of isotype switching. Also known as: down regulation of isotype switching, down-regulation of isotype switching, downregulation of isotype switching, negative regulation of class switch recombination, negative regulation of class switching, negative regulation of isotype switch recombination, inhibition of isotype switching